{
  "gene": "UniProtKB:H0YKK7",
  "gene_name": "Putative golgin subfamily A member 6-like protein 19",
  "term_id": "UNKNOWN:0002",
  "term_label": "Unknown biological process",
  "gene_symbol": "GOLGA6L19"
}